RNA polymerase II CTD heptapeptide repeat S2 kinase activity [GO:0140834] (molecular function) Also known as: RNA polymerase II C-terminal domain S2 kinase activity Definition: Catalysis of the reaction: ATP + RNA polymerase II large subunit CTD heptapeptide repeat (consensus YSPTSPS) = ADP + H+ + RNA polymerase II large subunit phosphoserine (position 2). Relationships: is a type of RNA polymerase II CTD heptapeptide repeat kinase activity [GO:0008353] References: PMID:28248323